{
  "term_label": "microtubule-based movement",
  "gene_symbol": "DYNLT2",
  "gene_name": "Dynein light chain Tctex-type protein 2",
  "term_id": "GO:0007018",
  "gene": "UniProtKB:Q8IZS6"
}